{
  "term_label": "intermembrane lipid transfer",
  "term_id": "GO:0120009",
  "gene": "UniProtKB:Q9Y5P4",
  "gene_symbol": "CERT1",
  "gene_name": "Ceramide transfer protein"
}